rDNA protrusion [GO:0030875] (cellular component) Note: Note that this component is characterized in Schizosaccharomyces, particularly with respect to the DAPI staining pattern. References: PMID:1629244 Definition: Any of the tandem arrays of rDNA localized at the periphery of the nucleus and protruding into the nucleolus, and associated proteins. May be visible as a single or double spot by DAPI staining. Relationships: is a type of cellular anatomical structure [GO:0110165]; is part of nucleolar chromatin [GO:0030874] Also known as: ribosomal DNA protrusion